{
  "gene_name": "Sterile alpha motif domain-containing protein 9",
  "gene": "UniProtKB:Q5K651",
  "term_label": "Unknown molecular function",
  "gene_symbol": "SAMD9",
  "term_id": "UNKNOWN:0001"
}